{
  "gene_symbol": "TTLL3",
  "gene": "UniProtKB:Q9Y4R7",
  "term_id": "GO:0035082",
  "gene_name": "Tubulin monoglycylase TTLL3",
  "term_label": "axoneme assembly"
}